{
  "term_id": "GO:0034446",
  "gene_name": "Paxillin",
  "gene": "UniProtKB:P49023",
  "term_label": "substrate adhesion-dependent cell spreading",
  "gene_symbol": "PXN"
}